{
  "term_label": "regulation of systemic arterial blood pressure by endothelin",
  "gene_symbol": "EDN2",
  "term_id": "GO:0003100",
  "gene_name": "Endothelin-2",
  "gene": "UniProtKB:P20800"
}